{
  "gene_name": "Ret finger protein-like 3",
  "gene_symbol": "RFPL3",
  "term_id": "GO:0010468",
  "gene": "UniProtKB:O75679",
  "term_label": "regulation of gene expression"
}